intracellular transport of viral protein in host cell [GO:0019060] (biological process) Note: This term is for annotation of proteins responsible for the movement of individual viral proteins, rather than the whole viral particle. Definition: The directed movement of a viral protein within the host cell. Also known as: intracellular transport of viral proteins in host cell, intracellular viral protein transport, cytoplasmic viral capsid transport, intracellular transport of viral capsid in host cell, intracellular transport of viral capsid protein in host cell, intracellular viral capsid transport, nuclear viral capsid transport, viral capsid transport in host cell cytoplasm, viral capsid transport in host cell nucleus References: PMID:11581394, PMID:9188566 Sources: GOC:ai, ISBN:0781702534, ISBN:0781718325 Relationships: is a type of symbiont intracellular protein transport in host [GO:0030581]; BFO_0000050 GO:0046719